somatic diversification of variable lymphocyte receptors of jawless fish [GO:0002202] (biological process) Note: Note that jawless fish refers to both lampreys (Petremyzontidae, ncbi_taxonomy_id:7746) and hagfish (Myxinidae, ncbi_taxonomy_id:7762). References: PMID:16373579 Sources: GOC:add Definition: The somatic process that results in the generation of sequence diversity of the variable lymphocyte receptors (VLR) of jawless fish. Relationships: is_a somatic diversification of immune receptors [GO:0002200]